{
  "gene_name": "Interleukin-17B",
  "gene": "UniProtKB:Q9UHF5",
  "gene_symbol": "IL17B",
  "term_id": "UNKNOWN:0001",
  "term_label": "Unknown molecular function"
}